positive regulation of substance P secretion [GO:1904460] (biological process) Also known as: up regulation of substance P secretion, up-regulation of substance P secretion, upregulation of substance P secretion, activation of substance P secretion Relationships: is a type of positive regulation of peptide hormone secretion [GO:0090277]; is_a regulation of substance P secretion [GO:1904458]; positively regulates substance P secretion [GO:1990772] References: PMID:11278900 Sources: GOC:TermGenie, GO_REF:0000058 Definition: Any process that activates or increases the frequency, rate or extent of substance P secretion. Subtypes: positive regulation of substance P secretion, neurotransmission [GO:1904496]